{
  "term_label": "mitochondrion",
  "gene_symbol": "FMC1",
  "gene": "UniProtKB:Q96HJ9",
  "gene_name": "Protein FMC1 homolog",
  "term_id": "GO:0005739"
}